{
  "term_label": "early endosome membrane",
  "gene_symbol": "MARCHF8",
  "gene_name": "E3 ubiquitin-protein ligase MARCHF8",
  "term_id": "GO:0031901",
  "gene": "UniProtKB:Q5T0T0"
}